{
  "gene": "UniProtKB:Q6P9A2",
  "gene_name": "Polypeptide N-acetylgalactosaminyltransferase 18",
  "term_label": "polypeptide N-acetylgalactosaminyltransferase activity",
  "term_id": "GO:0004653",
  "gene_symbol": "GALNT18"
}